{
  "gene": "UniProtKB:Q86SS6",
  "term_label": "positive regulation of vesicle fusion",
  "gene_name": "Synaptotagmin-9",
  "term_id": "GO:0031340",
  "gene_symbol": "SYT9"
}